symbiont-mediated perturbation of host cell cycle progression [GO:0044071] (biological process) Sources: MITRE:tk Definition: A process in which a symbiont interferes with the normal progression through the host cell cycle. The host is defined as the larger of the organisms involved in a symbiotic interaction. Subtypes: GO:0039592, symbiont-mediated perturbation of host exit from mitosis [GO:0039593], symbiont-mediated perturbation of host cell cycle G1/S transition checkpoint [GO:0039645] Relationships: is a type of symbiont-mediated perturbation of host cellular process [GO:0044068] Also known as: modification by symbiont of host cell cycle, modulation by symbiont of host cell cycle, modulation of host cell cycle by symbiont, perturbation of host cell cycle progression, regulation by symbiont of host cell cycle